regulation of mRNA export from nucleus in response to heat stress [GO:2000728] (biological process) Also known as: regulation of mRNA export from cell nucleus during heat stress, regulation of mRNA export from nucleus during heat stress Definition: Any process that modulates the frequency, rate or extent of mRNA export from nucleus in response to heat stress. References: PMID:15210706 Relationships: is_a regulation of mRNA export from nucleus [GO:0010793]; is a type of GO:1900034; regulates GO:0031990